{
  "gene_symbol": "ZSCAN5B",
  "term_label": "RNA polymerase II cis-regulatory region sequence-specific DNA binding",
  "gene": "UniProtKB:A6NJL1",
  "gene_name": "Zinc finger and SCAN domain-containing protein 5B",
  "term_id": "GO:0000978"
}